{
  "gene": "UniProtKB:P61018",
  "term_label": "GTPase activity",
  "gene_symbol": "RAB4B",
  "gene_name": "Ras-related protein Rab-4B",
  "term_id": "GO:0003924"
}